regulation of tetrapyrrole biosynthetic process [GO:1901463] (biological process) Definition: Any process that modulates the frequency, rate or extent of tetrapyrrole biosynthetic process. Sources: GOC:TermGenie, GOC:mengo_curators Also known as: regulation of tetrapyrrole anabolism, regulation of tetrapyrrole biosynthesis, regulation of tetrapyrrole formation, regulation of tetrapyrrole synthesis Relationships: is a type of GO:0009889; is a type of regulation of tetrapyrrole metabolic process [GO:1901401]; regulates tetrapyrrole biosynthetic process [GO:0033014] Subtypes: GO:0010380, GO:0070453, regulation of tetrapyrrole biosynthetic process from glutamate [GO:1901410], regulation of tetrapyrrole biosynthetic process from glycine and succinyl-CoA [GO:1901413], GO:1901464, positive regulation of tetrapyrrole biosynthetic process [GO:1901465]